protein lipoylation [GO:0009249] (BP) Sources: RESID:AA0118 Definition: The lipoylation of peptidyl-lysine to form peptidyl-N6-lipoyl-L-lysine. Also known as: peptidyl-lysine lipoylation, protein-lipoic acid cofactor linkage Relationships: is a type of peptidyl-lysine modification [GO:0018205]; is a type of protein maturation [GO:0051604]